{
  "gene_symbol": "ATP1A4",
  "gene": "UniProtKB:Q13733",
  "gene_name": "Sodium_potassium-transporting ATPase subunit alpha-4",
  "term_id": "GO:0036376",
  "term_label": "sodium ion export across plasma membrane"
}